{
  "gene": "UniProtKB:P02656",
  "gene_name": "Apolipoprotein C-III",
  "term_label": "intermediate-density lipoprotein particle",
  "term_id": "GO:0034363",
  "gene_symbol": "APOC3"
}